{
  "gene_symbol": "SPG11",
  "gene_name": "Spatacsin",
  "term_id": "GO:0008088",
  "gene": "UniProtKB:Q96JI7",
  "term_label": "axo-dendritic transport"
}